{
  "gene": "UniProtKB:Q96AV8",
  "gene_symbol": "E2F7",
  "term_label": "RNA polymerase II cis-regulatory region sequence-specific DNA binding",
  "gene_name": "Transcription factor E2F7",
  "term_id": "GO:0000978"
}